{
  "term_id": "UNKNOWN:0001",
  "gene_name": "Testis-expressed protein 53",
  "term_label": "Unknown molecular function",
  "gene": "UniProtKB:A0A1B0GU33",
  "gene_symbol": "TEX53"
}